chordate embryonic development [GO:0043009] (biological process) Definition: The process whose specific outcome is the progression of the embryo over time, from zygote formation through a stage including a notochord and neural tube until birth or egg hatching. Sources: GOC:mtg_sensu Relationships: is a type of embryo development ending in birth or egg hatching [GO:0009792] Subtypes: in utero embryonic development [GO:0001701]